{
  "gene_name": "DBF4-type zinc finger-containing protein 2",
  "term_id": "GO:0071514",
  "term_label": "genomic imprinting",
  "gene_symbol": "ZDBF2",
  "gene": "UniProtKB:Q9HCK1"
}